{
  "term_id": "GO:0005912",
  "gene": "UniProtKB:Q9NQS3",
  "gene_name": "Nectin-3",
  "term_label": "adherens junction",
  "gene_symbol": "NECTIN3"
}